{
  "term_label": "Unknown biological process",
  "gene": "UniProtKB:Q8IXR9",
  "term_id": "UNKNOWN:0002",
  "gene_symbol": "C12orf56",
  "gene_name": "Uncharacterized protein C12orf56"
}